{
  "term_id": "GO:0005737",
  "gene": "UniProtKB:P27144",
  "term_label": "cytoplasm",
  "gene_symbol": "AK4",
  "gene_name": "Adenylate kinase 4, mitochondrial"
}